positive regulation of cardiac muscle fiber development [GO:0055020] (BP) Relationships: is a type of positive regulation of cell development [GO:0010720]; is a type of regulation of cardiac muscle fiber development [GO:0055018]; is a type of positive regulation of cardiac muscle cell differentiation [GO:2000727]; positively regulates cardiac muscle cell development [GO:0055013] Also known as: positive regulation of cardiac muscle fibre development, positive regulation of heart muscle fiber development, up regulation of cardiac muscle fiber development, up-regulation of cardiac muscle fiber development, upregulation of cardiac muscle fiber development, activation of cardiac muscle fiber development, stimulation of cardiac muscle fiber development Definition: Any process that activates, maintains or increases the frequency, rate or extent of cardiac muscle fiber development. Sources: GOC:vk